{
  "gene": "UniProtKB:P35346",
  "term_label": "cellular response to glucocorticoid stimulus",
  "gene_name": "Somatostatin receptor type 5",
  "term_id": "GO:0071385",
  "gene_symbol": "SSTR5"
}